type 6 metabotropic glutamate receptor binding [GO:0031803] (molecular function) Sources: GOC:mah, GOC:nln Definition: Binding to a type 6 metabotropic glutamate receptor. Relationships: is a type of GO:0035256 Also known as: type 6 metabotropic glutamate receptor ligand